{
  "term_label": "vesicle-mediated transport",
  "term_id": "GO:0016192",
  "gene_name": "Synaptotagmin-15",
  "gene": "UniProtKB:Q9BQS2",
  "gene_symbol": "SYT15"
}